intrinsic apoptotic signaling pathway in response to nitrosative stress [GO:1990442] (biological process) Regulation: regulated by regulation of nitrosative stress-induced intrinsic apoptotic signaling pathway [GO:1905258]; negatively regulated by GO:1905259; positively regulated by positive regulation of nitrosative stress-induced intrinsic apoptotic signaling pathway [GO:1905260] References: PMID:23985028 Sources: GOC:PARL, GOC:bf Relationships: is a type of GO:0071500; is a type of intrinsic apoptotic signaling pathway [GO:0097193] Also known as: nitrosative stress-induced intrinsic apoptotic signaling pathway, nitrosative stress-induced apoptosis Definition: The series of molecular signals in which an intracellular signal is conveyed to trigger the apoptotic death of a cell. The pathway is induced in response to nitrosative stress; a state often resulting from exposure to high levels of nitric oxide (NO) or the highly reactive oxidant peroxynitrite, which is produced following interaction of NO with superoxide anions.